{
  "gene": "UniProtKB:Q9H299",
  "gene_symbol": "SH3BGRL3",
  "term_id": "GO:0007010",
  "term_label": "cytoskeleton organization",
  "gene_name": "SH3 domain-binding glutamic acid-rich-like protein 3"
}